protein-carbohydrate complex [GO:0032992] (cellular component) Subtypes: GO:0071666 Sources: GOC:mah Relationships: is a type of protein-containing complex [GO:0032991] Note: Macromolecular complexes in which the carbohydrate component is all covalently bound to protein are not considered protein carbohydrate complexes. Definition: A macromolecular complex containing separate protein and carbohydrate molecules. Separate in this context means not covalently bound to each other.